{
  "term_label": "neuropeptide binding",
  "term_id": "GO:0042923",
  "gene_symbol": "SSTR5",
  "gene_name": "Somatostatin receptor type 5",
  "gene": "UniProtKB:P35346"
}